{
  "term_id": "UNKNOWN:0003",
  "gene": "UniProtKB:Q7Z2Q7",
  "gene_name": "Leucine-rich repeat-containing protein 70",
  "term_label": "Unknown cellular component",
  "gene_symbol": "LRRC70"
}